{
  "gene_name": "Zinc finger protein 30",
  "gene": "UniProtKB:P17039",
  "term_label": "DNA-binding transcription factor activity, RNA polymerase II-specific",
  "gene_symbol": "ZNF30",
  "term_id": "GO:0000981"
}